{
  "gene_name": "Actin-related protein 2",
  "gene": "UniProtKB:P61160",
  "term_id": "GO:0034314",
  "gene_symbol": "ACTR2",
  "term_label": "Arp2/3 complex-mediated actin nucleation"
}